{
  "term_id": "GO:0008135",
  "gene_name": "Cytoplasmic polyadenylation element-binding protein 1",
  "gene_symbol": "CPEB1",
  "term_label": "translation factor activity, RNA binding",
  "gene": "UniProtKB:Q9BZB8"
}